cobalt-precorrin-8 methylmutase activity [GO:0043778] (molecular function) Relationships: is a type of GO:0016867 Sources: MetaCyc:RXN-8768 Also known as: cobalt-precorrin 8 methylmutase activity, cobalt-precorrin 8X methylmutase activity, cobalt-precorrin-8X methylmutase activity Definition: Catalysis of the reaction: cobalt-precorrin 8 = cobyrinate.